{
  "gene": "UniProtKB:Q9HBX3",
  "term_label": "Unknown biological process",
  "term_id": "UNKNOWN:0002",
  "gene_name": "Uncharacterized protein encoded by SND1-IT1",
  "gene_symbol": "SND1-IT1"
}